NAE1-UBA3 complex [GO:0120500] (cellular component) References: PMID:12740388, PMID:21931660 Also known as: APPBP1-UBA3 complex, NAE, NEDD8 activating enzyme Relationships: is a type of catalytic complex [GO:1902494] Definition: A heterodimeric E1 complex that activates the ubiquitin-like protein NEDD8. In humans the subunits are NAE1 (also known as APPBP1) and UBA3.